immune response involved in response to exogenous dsRNA [GO:1902615] (biological process) Definition: Any immune response that is involved in response to exogenous dsRNA. Relationships: is a type of immune response [GO:0006955]; is part of response to exogenous dsRNA [GO:0043330] References: PMID:21266579 Sources: GOC:TermGenie, GOC:pg, GO_REF:0000060 Also known as: immune response involved in response to exogenous double-stranded RNA, immune response involved in response to viral dsRNA